{
  "gene_name": "Ral guanine nucleotide dissociation stimulator-like 2",
  "term_label": "Unknown biological process",
  "gene_symbol": "RGL2",
  "term_id": "UNKNOWN:0002",
  "gene": "UniProtKB:O15211"
}